cellular response to luteinizing hormone stimulus [GO:0071373] (biological process) Definition: Any process that results in a change in state or activity of a cell (in terms of movement, secretion, enzyme production, gene expression, etc.) as a result of a luteinizing hormone stimulus. Sources: GOC:mah Relationships: is_a response to luteinizing hormone [GO:0034699]; is a type of cellular response to gonadotropin stimulus [GO:0071371]; is a type of cellular response to peptide hormone stimulus [GO:0071375]